{
  "gene_symbol": "TOR1AIP1",
  "term_label": "nuclear membrane",
  "term_id": "GO:0031965",
  "gene": "UniProtKB:Q5JTV8",
  "gene_name": "Torsin-1A-interacting protein 1"
}